{
  "gene_name": "Protein arginine N-methyltransferase 6",
  "gene_symbol": "PRMT6",
  "term_label": "protein-arginine N-methyltransferase activity",
  "term_id": "GO:0016274",
  "gene": "UniProtKB:Q96LA8"
}